{
  "gene_symbol": "OMP",
  "term_label": "nucleus",
  "term_id": "GO:0005634",
  "gene": "UniProtKB:P47874",
  "gene_name": "Olfactory marker protein"
}